{
  "term_label": "chromosome",
  "gene_name": "Serine_threonine-protein kinase ATR",
  "gene_symbol": "ATR",
  "term_id": "GO:0005694",
  "gene": "UniProtKB:Q13535"
}